negative regulation of transcription from RNA polymerase II promoter by a nonfermentable carbon source [GO:0061415] (biological process) References: PMID:19686338 Sources: GOC:dph Definition: A transcription regulation process in which the presence of a nonfermentable carbon source leads to a decrease of the frequency, rate, or extent of transcription, from an RNA polymerase II promoter, of specific genes involved in the metabolism of other carbon sources. Relationships: is a type of carbon catabolite repression of transcription from RNA polymerase II promoter [GO:0000437]; is_a GO:0061413